{
  "gene_symbol": "DDX6",
  "gene": "UniProtKB:P26196",
  "term_label": "cytoplasmic stress granule",
  "term_id": "GO:0010494",
  "gene_name": "Probable ATP-dependent RNA helicase DDX6"
}